{
  "gene_name": "Vasopressin V1a receptor",
  "term_label": "positive regulation of vasoconstriction",
  "gene": "UniProtKB:P37288",
  "term_id": "GO:0045907",
  "gene_symbol": "AVPR1A"
}